{
  "gene": "UniProtKB:O60318",
  "gene_symbol": "MCM3AP",
  "term_label": "cytoplasm",
  "gene_name": "Germinal-center associated nuclear protein",
  "term_id": "GO:0005737"
}